{
  "gene": "UniProtKB:Q14746",
  "term_id": "GO:0007030",
  "gene_name": "Conserved oligomeric Golgi complex subunit 2",
  "term_label": "Golgi organization",
  "gene_symbol": "COG2"
}